ocellus pigment biosynthetic process [GO:0008055] (biological process) Subtypes: ommochrome biosynthetic process [GO:0006727] References: PMID:15176085, PMID:18421706 Sources: GOC:ai Also known as: ocellus pigment anabolism, ocellus pigment biosynthesis, ocellus pigment formation, ocellus pigment synthesis Relationships: is a type of GO:0044550; is a type of pigment biosynthetic process [GO:0046148]; is a type of ocellus pigment metabolic process [GO:0046158] Definition: The chemical reactions and pathways resulting in the formation of ocellus pigments, general or particular coloring matter in living organisms, found or utilized in the ocellus, a minute simple eye found in many invertebrates.